{
  "term_label": "Unknown molecular function",
  "gene_name": "Meiosis-specific nuclear structural protein 1",
  "gene_symbol": "MNS1",
  "gene": "UniProtKB:Q8NEH6",
  "term_id": "UNKNOWN:0001"
}